{
  "gene_name": "Myc proto-oncogene protein",
  "term_id": "GO:0008284",
  "gene_symbol": "MYC",
  "gene": "UniProtKB:P01106",
  "term_label": "positive regulation of cell population proliferation"
}